{
  "term_id": "UNKNOWN:0003",
  "gene_name": "Intermembrane lipid transfer protein VPS13B",
  "term_label": "Unknown cellular component",
  "gene": "UniProtKB:Q7Z7G8",
  "gene_symbol": "VPS13B"
}